{
  "gene_symbol": "MCM5",
  "term_label": "3'-5' DNA helicase activity",
  "gene_name": "DNA replication licensing factor MCM5",
  "term_id": "GO:0043138",
  "gene": "UniProtKB:P33992"
}